{
  "gene_symbol": "CGB2",
  "term_id": "GO:0005615",
  "gene": "UniProtKB:Q6NT52",
  "gene_name": "Choriogonadotropin subunit beta variant 2",
  "term_label": "extracellular space"
}